mating projection actin fusion focus assembly [GO:1904600] (biological process) Also known as: actin fusion focus assembly, actin fusion focus formation Relationships: is a type of cellular component assembly involved in morphogenesis [GO:0010927]; is a type of actin cytoskeleton organization [GO:0030036]; is part of mating projection formation [GO:0031382] References: PMID:25825517 Sources: GOC:TermGenie, GO_REF:0000079 Definition: The aggregation, arrangement and bonding together of a set of components to form an actin fusion focus.